{
  "term_id": "GO:0005886",
  "gene_name": "Olfactory receptor 3A2",
  "gene_symbol": "OR3A2",
  "term_label": "plasma membrane",
  "gene": "UniProtKB:P47893"
}